{
  "term_label": "centrosome",
  "term_id": "GO:0005813",
  "gene_symbol": "CKAP2L",
  "gene": "UniProtKB:Q8IYA6",
  "gene_name": "Cytoskeleton-associated protein 2-like"
}